{
  "gene_name": "Zinc finger FYVE domain-containing protein 16",
  "gene": "UniProtKB:Q7Z3T8",
  "gene_symbol": "ZFYVE16",
  "term_id": "GO:0031901",
  "term_label": "early endosome membrane"
}